{
  "gene": "UniProtKB:Q8N1B4",
  "gene_name": "Vacuolar protein sorting-associated protein 52 homolog",
  "term_label": "GARP complex",
  "gene_symbol": "VPS52",
  "term_id": "GO:0000938"
}